{
  "gene_name": "Protein RFT1 homolog",
  "gene_symbol": "RFT1",
  "term_label": "Unknown molecular function",
  "gene": "UniProtKB:Q96AA3",
  "term_id": "UNKNOWN:0001"
}